{
  "term_label": "Unknown biological process",
  "gene": "UniProtKB:Q8NGL7",
  "gene_name": "Olfactory receptor 4P4",
  "term_id": "UNKNOWN:0002",
  "gene_symbol": "OR4P4"
}